negative regulation of chronic inflammatory response to non-antigenic stimulus [GO:0002881] (biological process) Relationships: is a type of GO:0002677; is a type of regulation of chronic inflammatory response to non-antigenic stimulus [GO:0002880]; negatively regulates chronic inflammatory response to non-antigenic stimulus [GO:0002545] Sources: GOC:add Definition: Any process that stops, prevents, or reduces the frequency, rate, or extent of a chronic inflammatory response to a non-antigenic stimulus. Also known as: down regulation of chronic inflammatory response to non-antigenic stimulus, down-regulation of chronic inflammatory response to non-antigenic stimulus, downregulation of chronic inflammatory response to non-antigenic stimulus, inhibition of chronic inflammatory response to non-antigenic stimulus